{
  "term_label": "negative regulation of cAMP/PKA signal transduction",
  "term_id": "GO:0141162",
  "gene_name": "High affinity cAMP-specific 3',5'-cyclic phosphodiesterase 7A",
  "gene_symbol": "PDE7A",
  "gene": "UniProtKB:Q13946"
}